{
  "term_id": "GO:0036128",
  "gene": "UniProtKB:Q9NTU4",
  "term_label": "CatSper complex",
  "gene_symbol": "CATSPERZ",
  "gene_name": "Cation channel sperm-associated auxiliary subunit zeta"
}